{
  "gene_name": "S-acyl fatty acid synthase thioesterase, medium chain",
  "term_id": "GO:0008610",
  "gene": "UniProtKB:Q9NV23",
  "term_label": "lipid biosynthetic process",
  "gene_symbol": "OLAH"
}